{
  "gene_name": "Homeobox protein SIX2",
  "gene_symbol": "SIX2",
  "term_id": "GO:0006357",
  "gene": "UniProtKB:Q9NPC8",
  "term_label": "regulation of transcription by RNA polymerase II"
}